{
  "gene": "UniProtKB:Q5SZI1",
  "term_id": "UNKNOWN:0002",
  "gene_symbol": "LDLRAD2",
  "term_label": "Unknown biological process",
  "gene_name": "Low-density lipoprotein receptor class A domain-containing protein 2"
}